{
  "gene_name": "Hydroxylysine kinase",
  "gene": "UniProtKB:A2RU49",
  "term_id": "UNKNOWN:0002",
  "gene_symbol": "HYKK",
  "term_label": "Unknown biological process"
}